{
  "term_label": "Unknown cellular component",
  "gene_name": "Zinc finger protein with KRAB and SCAN domains 2",
  "gene": "UniProtKB:Q63HK3",
  "term_id": "UNKNOWN:0003",
  "gene_symbol": "ZKSCAN2"
}